{
  "term_label": "plasma membrane",
  "gene_symbol": "A1BG",
  "gene": "UniProtKB:P04217",
  "gene_name": "Alpha-1B-glycoprotein",
  "term_id": "GO:0005886"
}